{
  "term_label": "Unknown biological process",
  "gene": "UniProtKB:A2RU37",
  "gene_symbol": "LINC02872",
  "term_id": "UNKNOWN:0002",
  "gene_name": "Uncharacterized protein encoded by LINC02872"
}